NAD+-protein-histidine ADP-ribosyltransferase activity [GO:0140815] (molecular function) Relationships: is a type of NAD+-protein mono-ADP-ribosyltransferase activity [GO:1990404] References: PMID:35393539 Sources: RHEA:72071 Definition: Catalysis of the reaction: L-histidyl-[protein] + NAD+ = H+ + Nt-(ADP-D-ribosyl)-L-histidyl-[protein] + nicotinamide.